serotonergic neuron axon guidance [GO:0036515] (biological process) Relationships: is a type of axon guidance [GO:0007411] Definition: The chemotaxis process that directs the migration of an axon growth cone of a serotonergic neuron to a specific target site in response to a combination of attractive and repulsive cues. References: PMID:21106844 Sources: CL:0000850, GOC:PARL, GOC:bf Also known as: 5-HT axon guidance, serotonergic axon guidance